{
  "term_label": "intermediate filament",
  "gene": "UniProtKB:Q9UPN3",
  "term_id": "GO:0005882",
  "gene_symbol": "MACF1",
  "gene_name": "Microtubule-actin cross-linking factor 1, isoforms 1_2_3_4_5"
}